{
  "term_id": "GO:0042802",
  "gene": "UniProtKB:Q8TDQ7",
  "gene_name": "Glucosamine-6-phosphate isomerase 2",
  "term_label": "identical protein binding",
  "gene_symbol": "GNPDA2"
}